{
  "gene": "UniProtKB:Q9HB03",
  "term_id": "GO:0019367",
  "term_label": "fatty acid elongation, saturated fatty acid",
  "gene_symbol": "ELOVL3",
  "gene_name": "Elongation of very long chain fatty acids protein 3"
}